{
  "term_label": "microfibril",
  "term_id": "GO:0001527",
  "gene_symbol": "MFAP5",
  "gene": "UniProtKB:Q13361",
  "gene_name": "Microfibrillar-associated protein 5"
}